{
  "gene_name": "XK-related protein 9",
  "term_label": "Unknown molecular function",
  "term_id": "UNKNOWN:0001",
  "gene_symbol": "XKR9",
  "gene": "UniProtKB:Q5GH70"
}